{
  "gene_name": "Valine--tRNA ligase",
  "term_id": "GO:0005829",
  "term_label": "cytosol",
  "gene": "UniProtKB:P26640",
  "gene_symbol": "VARS1"
}